lactone metabolic process [GO:1901334] (biological process) Definition: The chemical reactions and pathways involving lactone. Relationships: is a type of metabolic process [GO:0008152] Sources: GOC:TermGenie Also known as: lactone metabolism Subtypes: L-ascorbic acid metabolic process [GO:0019852], GO:0033067, lactone catabolic process [GO:1901335], lactone biosynthetic process [GO:1901336], GO:1901600